{
  "term_label": "natural killer cell lectin-like receptor binding",
  "term_id": "GO:0046703",
  "gene": "UniProtKB:Q9BZM4",
  "gene_symbol": "ULBP3",
  "gene_name": "UL16-binding protein 3"
}